{
  "gene_symbol": "ARHGAP27",
  "gene": "UniProtKB:Q6ZUM4",
  "gene_name": "Rho GTPase-activating protein 27",
  "term_label": "cytoplasm",
  "term_id": "GO:0005737"
}